{
  "gene_symbol": "RNF41",
  "gene": "UniProtKB:Q9H4P4",
  "gene_name": "E3 ubiquitin-protein ligase NRDP1",
  "term_id": "GO:0006511",
  "term_label": "ubiquitin-dependent protein catabolic process"
}